primary shoot apical meristem specification [GO:0010072] (BP) Sources: GOC:ascb_2009, GOC:dph, GOC:tair_curators, GOC:tb Definition: The specification of the meristem which will give rise to all post-embryonic above-ground structures of the plant as well as the non-root below-ground structures, such as rhizomes and tubers. Also known as: embryo shoot apical meristem specification Relationships: is a type of developmental process involved in reproduction [GO:0003006]; is a type of embryonic meristem initiation [GO:0090421]; is part of shoot system morphogenesis [GO:0010016]; is part of embryonic meristem development [GO:0048508]